{
  "gene": "UniProtKB:Q9NX09",
  "term_id": "GO:0001666",
  "gene_name": "DNA damage-inducible transcript 4 protein",
  "gene_symbol": "DDIT4",
  "term_label": "response to hypoxia"
}